{
  "term_label": "plasma membrane",
  "gene_name": "T cell receptor beta chain MC.7.G5",
  "gene": "UniProtKB:P0DTU4",
  "term_id": "GO:0005886",
  "gene_symbol": "TRB"
}